{
  "term_label": "bicarbonate transport",
  "gene_symbol": "CFTR",
  "gene": "UniProtKB:P13569",
  "gene_name": "Cystic fibrosis transmembrane conductance regulator",
  "term_id": "GO:0015701"
}